{
  "gene_name": "Transcription factor SOX-18",
  "gene": "UniProtKB:P35713",
  "term_id": "GO:0005634",
  "term_label": "nucleus",
  "gene_symbol": "SOX18"
}